{
  "gene_name": "Thymus-specific serine protease",
  "gene": "UniProtKB:Q9NQE7",
  "term_label": "Unknown biological process",
  "term_id": "UNKNOWN:0002",
  "gene_symbol": "PRSS16"
}